{
  "gene_symbol": "STXBP2",
  "gene_name": "Syntaxin-binding protein 2",
  "gene": "UniProtKB:Q15833",
  "term_label": "intracellular protein transport",
  "term_id": "GO:0006886"
}